{
  "term_id": "GO:0016887",
  "gene_name": "DNA mismatch repair protein Mlh3",
  "term_label": "ATP hydrolysis activity",
  "gene": "UniProtKB:Q9UHC1",
  "gene_symbol": "MLH3"
}